{
  "term_id": "UNKNOWN:0003",
  "gene_name": "Acireductone dioxygenase",
  "gene": "UniProtKB:Q9BV57",
  "term_label": "Unknown cellular component",
  "gene_symbol": "ADI1"
}